{
  "term_id": "GO:0015187",
  "gene_name": "Proton-coupled amino acid transporter 3",
  "gene": "UniProtKB:Q495N2",
  "gene_symbol": "SLC36A3",
  "term_label": "glycine transmembrane transporter activity"
}